{
  "gene_name": "Kinesin-like protein KIF18A",
  "term_id": "GO:0005871",
  "gene_symbol": "KIF18A",
  "gene": "UniProtKB:Q8NI77",
  "term_label": "kinesin complex"
}